{
  "term_id": "GO:0042393",
  "gene_symbol": "A8MVJ9",
  "gene": "UniProtKB:A8MVJ9",
  "term_label": "histone binding",
  "gene_name": "Putative histone PARylation factor 1-like"
}